{
  "gene_symbol": "NDE1",
  "term_id": "GO:0008017",
  "gene": "UniProtKB:Q9NXR1",
  "gene_name": "Nuclear distribution protein nudE homolog 1",
  "term_label": "microtubule binding"
}